{
  "term_label": "maturation of LSU-rRNA from tricistronic rRNA transcript (SSU-rRNA, 5.8S rRNA, LSU-rRNA)",
  "gene": "UniProtKB:P42696",
  "term_id": "GO:0000463",
  "gene_name": "RNA-binding protein 34",
  "gene_symbol": "RBM34"
}